{
  "term_id": "GO:0005021",
  "gene_symbol": "FLT1",
  "term_label": "vascular endothelial growth factor receptor activity",
  "gene": "UniProtKB:P17948",
  "gene_name": "Vascular endothelial growth factor receptor 1"
}